{
  "term_id": "UNKNOWN:0003",
  "gene": "UniProtKB:Q9H628",
  "gene_name": "Ras-related and estrogen-regulated growth inhibitor-like protein",
  "gene_symbol": "RERGL",
  "term_label": "Unknown cellular component"
}